{
  "term_label": "neuronal cell body",
  "gene_symbol": "KCNN3",
  "term_id": "GO:0043025",
  "gene_name": "Small conductance calcium-activated potassium channel protein 3",
  "gene": "UniProtKB:Q9UGI6"
}